fatty acid beta-oxidation, unsaturated, even number [GO:0033542] (biological process) Subtypes: GO:0033543, fatty acid beta-oxidation, unsaturated, even number, epimerase pathway [GO:0033544] Relationships: is_a fatty acid beta-oxidation [GO:0006635] Definition: A fatty acid beta-oxidation pathway by which fatty acids having cis-double bonds on even-numbered carbons are degraded. Fatty acid beta-oxidation begins with the addition of coenzyme A to a fatty acid, and ends when only two or three carbons remain (as acetyl-CoA or propionyl-CoA respectively). Sources: GOC:mah, MetaCyc:PWY-5138